{
  "term_label": "cytoplasmic microtubule organization",
  "gene_symbol": "CLIP3",
  "gene": "UniProtKB:Q96DZ5",
  "gene_name": "CAP-Gly domain-containing linker protein 3",
  "term_id": "GO:0031122"
}